{
  "term_id": "GO:0031966",
  "gene": "UniProtKB:A8MWL7",
  "gene_symbol": "TMEM14DP",
  "gene_name": "Transmembrane protein 14DP",
  "term_label": "mitochondrial membrane"
}